{
  "term_id": "UNKNOWN:0001",
  "gene_name": "Uncharacterized protein",
  "gene_symbol": "A0A669KB60",
  "gene": "UniProtKB:A0A669KB60",
  "term_label": "Unknown molecular function"
}